{
  "gene": "UniProtKB:Q9H9L3",
  "term_label": "RNA processing",
  "gene_symbol": "ISG20L2",
  "term_id": "GO:0006396",
  "gene_name": "Interferon-stimulated 20 kDa exonuclease-like 2"
}